{
  "gene_name": "TRAF3-interacting protein 1",
  "gene": "UniProtKB:Q8TDR0",
  "term_id": "GO:0005930",
  "term_label": "axoneme",
  "gene_symbol": "TRAF3IP1"
}